cellular response to nitrite [GO:0071250] (biological process) Definition: Any process that results in a change in state or activity of a cell (in terms of movement, secretion, enzyme production, gene expression, etc.) as a result of a nitrite stimulus. Sources: GOC:mah Relationships: is a type of GO:0080033; is a type of cellular response to oxygen-containing compound [GO:1901701]; is a type of GO:1902170